DNA recombinase auxiliary factor complex [GO:0120231] (CC) Relationships: is_a enzyme activator complex [GO:0150005] Also known as: DNA recombinase accessory factor complex, DNA recombinase activator complex References: PMID:32414915 Definition: A protein complex that binds to a recombinase and incrseases its activity.